{
  "gene": "UniProtKB:Q96QZ7",
  "gene_symbol": "MAGI1",
  "term_id": "UNKNOWN:0001",
  "term_label": "Unknown molecular function",
  "gene_name": "Membrane-associated guanylate kinase, WW and PDZ domain-containing protein 1"
}